{
  "term_id": "GO:0005332",
  "gene": "UniProtKB:P31641",
  "gene_symbol": "SLC6A6",
  "gene_name": "Sodium- and chloride-dependent taurine transporter",
  "term_label": "gamma-aminobutyric acid:sodium:chloride symporter activity"
}